fibroblast activation [GO:0072537] (biological process) Sources: CL:0000057, GOC:BHF, GOC:mah Definition: A change in the morphology or behavior of a fibroblast resulting from exposure to an activating factor such as a cellular or soluble ligand. Relationships: is a type of cell activation [GO:0001775] Subtypes: hepatic stellate cell activation [GO:0035733]